{
  "gene": "UniProtKB:P31267",
  "term_id": "GO:0006357",
  "gene_symbol": "HOXA6",
  "term_label": "regulation of transcription by RNA polymerase II",
  "gene_name": "Homeobox protein Hox-A6"
}